{
  "term_id": "GO:0050253",
  "gene_symbol": "PLB1",
  "gene": "UniProtKB:Q6P1J6",
  "term_label": "retinyl-palmitate esterase activity",
  "gene_name": "Phospholipase B1, membrane-associated"
}